{
  "gene_name": "Galectin-9B",
  "gene": "UniProtKB:Q3B8N2",
  "term_id": "GO:2000562",
  "gene_symbol": "LGALS9B",
  "term_label": "negative regulation of CD4-positive, alpha-beta T cell proliferation"
}